{
  "gene_symbol": "THRB",
  "term_id": "GO:0005634",
  "gene": "UniProtKB:P10828",
  "gene_name": "Thyroid hormone receptor beta",
  "term_label": "nucleus"
}